negative regulation of filopodium assembly [GO:0051490] (biological process) Definition: Any process that stops, prevents, or reduces the frequency, rate or extent of the assembly of a filopodium, a thin, stiff protrusion extended by the leading edge of a motile cell such as a crawling fibroblast or amoeba, or an axonal growth cone. Sources: GOC:ai Also known as: down regulation of filopodium formation, down-regulation of filopodium formation, downregulation of filopodium formation, negative regulation of filopodia biosynthesis, negative regulation of filopodia formation, negative regulation of filopodium formation, inhibition of filopodium formation Relationships: is a type of regulation of filopodium assembly [GO:0051489]; is a type of negative regulation of plasma membrane bounded cell projection assembly [GO:0120033]; negatively regulates filopodium assembly [GO:0046847]